{
  "term_label": "nucleus",
  "gene_symbol": "NLK",
  "term_id": "GO:0005634",
  "gene": "UniProtKB:Q9UBE8",
  "gene_name": "Serine_threonine-protein kinase NLK"
}